positive regulation of DNA repair [GO:0045739] (biological process) Definition: Any process that activates or increases the frequency, rate or extent of DNA repair. Sources: GOC:go_curators Also known as: up regulation of DNA repair, up-regulation of DNA repair, upregulation of DNA repair, activation of DNA repair, stimulation of DNA repair Relationships: is a type of regulation of DNA repair [GO:0006282]; is a type of positive regulation of response to stimulus [GO:0048584]; is_a GO:0051054; positively regulates DNA repair [GO:0006281] Subtypes: positive regulation of mismatch repair [GO:0032425], GO:1903518, positive regulation of base-excision repair [GO:1905053], positive regulation of double-strand break repair [GO:2000781]